{
  "gene_name": "Transcription factor Dp-2",
  "term_id": "GO:0006357",
  "gene_symbol": "TFDP2",
  "gene": "UniProtKB:Q14188",
  "term_label": "regulation of transcription by RNA polymerase II"
}